{
  "term_id": "GO:0006955",
  "gene_name": "Immunoglobulin lambda variable 1-36",
  "term_label": "immune response",
  "gene_symbol": "IGLV1-36",
  "gene": "UniProtKB:A0A0B4J1U3"
}